{
  "gene_name": "Iroquois-class homeodomain protein IRX-4",
  "gene_symbol": "IRX4",
  "gene": "UniProtKB:P78413",
  "term_label": "neuron differentiation",
  "term_id": "GO:0030182"
}